{
  "gene_name": "Transcription initiation factor IIB",
  "term_id": "GO:0001174",
  "term_label": "transcriptional start site selection at RNA polymerase II promoter",
  "gene": "UniProtKB:Q00403",
  "gene_symbol": "GTF2B"
}